{
  "gene_name": "Axin-2",
  "term_label": "positive regulation of proteasomal ubiquitin-dependent protein catabolic process",
  "term_id": "GO:0032436",
  "gene_symbol": "AXIN2",
  "gene": "UniProtKB:Q9Y2T1"
}